{
  "term_id": "UNKNOWN:0003",
  "gene": "UniProtKB:Q96BT3",
  "gene_name": "Centromere protein T",
  "gene_symbol": "CENPT",
  "term_label": "Unknown cellular component"
}